{
  "gene": "UniProtKB:P35225",
  "gene_name": "Interleukin-13",
  "gene_symbol": "IL13",
  "term_id": "GO:0005576",
  "term_label": "extracellular region"
}